rRNA (cytosine-2'-O-)-methyltransferase activity [GO:0070677] (molecular function) References: PMID:19400805 Sources: GOC:mah Relationships: is a type of GO:0016434; is a type of RNA 2'-O-methyltransferase activity [GO:0062105] Definition: Catalysis of the reaction: S-adenosyl-L-methionine + rRNA = S-adenosyl-L-homocysteine + rRNA containing 2'-O-methylcytosine.